negative regulation of filamentous growth of a population of unicellular organisms [GO:1900429] (biological process) Also known as: down regulation of filamentous growth of a population of unicellular organisms, down-regulation of filamentous growth of a population of unicellular organisms, downregulation of filamentous growth of a population of unicellular organisms, inhibition of filamentous growth of a population of unicellular organisms Sources: GOC:TermGenie, GOC:di Subtypes: negative regulation of growth of unicellular organism as a thread of attached cells [GO:0070785], negative regulation of filamentous growth of a population of unicellular organisms in response to heat [GO:1900432], negative regulation of filamentous growth of a population of unicellular organisms in response to chemical stimulus [GO:1900438], negative regulation of filamentous growth of a population of unicellular organisms in response to biotic stimulus [GO:1900444], GO:1900742 Definition: Any process that stops, prevents or reduces the frequency, rate or extent of filamentous growth of a population of unicellular organisms. Relationships: is a type of negative regulation of filamentous growth [GO:0060258]; is a type of regulation of filamentous growth of a population of unicellular organisms [GO:1900428]; negatively regulates filamentous growth of a population of unicellular organisms [GO:0044182]